{
  "term_label": "G protein-coupled receptor binding",
  "gene_name": "Rho guanine nucleotide exchange factor 11",
  "term_id": "GO:0001664",
  "gene": "UniProtKB:O15085",
  "gene_symbol": "ARHGEF11"
}